trigeminal nerve development [GO:0021559] (biological process) Relationships: is a type of cranial nerve development [GO:0021545] Definition: The process whose specific outcome is the progression of the trigeminal nerve over time, from its formation to the mature structure. The trigeminal nerve is composed of three large branches. They are the ophthalmic (V1, sensory), maxillary (V2, sensory) and mandibular (V3, motor and sensory) branches. The sensory ophthalmic branch travels through the superior orbital fissure and passes through the orbit to reach the skin of the forehead and top of the head. The maxillary nerve contains sensory branches that reach the pterygopalatine fossa via the inferior orbital fissure (face, cheek and upper teeth) and pterygopalatine canal (soft and hard palate, nasal cavity and pharynx). The motor part of the mandibular branch is distributed to the muscles of mastication, the mylohyoid muscle and the anterior belly of the digastric. The mandibular nerve also innervates the tensor veli palatini and tensor tympani muscles. The sensory part of the mandibular nerve is composed of branches that carry general sensory information from the mucous membranes of the mouth and cheek, anterior two-thirds of the tongue, lower teeth, skin of the lower jaw, side of the head and scalp and meninges of the anterior and middle cranial fossae. Also known as: cranial nerve 5 development, cranial nerve V development, CN V development Sources: GOC:cls, GOC:dgh, GOC:dph, GOC:jid, GO_REF:0000021